{
  "gene_name": "Tissue alpha-L-fucosidase",
  "term_id": "GO:0006004",
  "gene_symbol": "FUCA1",
  "gene": "UniProtKB:P04066",
  "term_label": "fucose metabolic process"
}